{
  "gene_symbol": "TMSB15B",
  "gene_name": "Thymosin beta-15B",
  "term_label": "protein sequestering activity",
  "term_id": "GO:0140311",
  "gene": "UniProtKB:P0CG35"
}